{
  "gene_symbol": "PCOLCE",
  "term_label": "Unknown cellular component",
  "gene_name": "Procollagen C-endopeptidase enhancer 1",
  "gene": "UniProtKB:Q15113",
  "term_id": "UNKNOWN:0003"
}